{
  "gene": "UniProtKB:Q5SRE7",
  "gene_name": "Phytanoyl-CoA dioxygenase domain-containing protein 1",
  "term_id": "UNKNOWN:0002",
  "gene_symbol": "PHYHD1",
  "term_label": "Unknown biological process"
}